{
  "term_label": "toxin metabolic process",
  "gene_symbol": "AS3MT",
  "term_id": "GO:0009404",
  "gene_name": "Arsenite methyltransferase",
  "gene": "UniProtKB:Q9HBK9"
}